hepoxilin-epoxide hydrolase activity [GO:0047977] (molecular function) Definition: Catalysis of the reaction: (5Z,9E,14Z)-(8x,11R,12S)-11,12-epoxy-8-hydroxyicosa-5,9,14-trienoate + H2O = (5Z,9E,14Z)-(8x,11x,12S)-8,11,12-trihydroxyicosa-5,9,14-trienoate. Also known as: (5Z,9E,14Z)-(8xi,11R,12S)-11,12-epoxy-8-hydroxyicosa-5,9,14-trienoate hydrolase activity, hepoxilin A(3) hydrolase activity, hepoxilin A3 hydrolase activity, hepoxilin epoxide hydrolase activity, hepoxylin hydrolase activity Sources: EC:3.3.2.7, MetaCyc:HEPOXILIN-EPOXIDE-HYDROLASE-RXN Relationships: is_a epoxide hydrolase activity [GO:0004301]